basipetal auxin transport [GO:0010540] (biological process) References: PMID:10677441 Definition: The unidirectional movement of auxin from the apex to base of an organ, including the shoot, leaf, primary root, or lateral root. Relationships: is_a auxin polar transport [GO:0009926]